{
  "gene": "UniProtKB:P35580",
  "gene_name": "Myosin-10",
  "gene_symbol": "MYH10",
  "term_id": "GO:0008360",
  "term_label": "regulation of cell shape"
}